{
  "gene_name": "High affinity immunoglobulin gamma Fc receptor I",
  "term_id": "GO:0009897",
  "gene": "UniProtKB:P12314",
  "term_label": "external side of plasma membrane",
  "gene_symbol": "FCGR1A"
}